diphthine methyl ester synthase activity [GO:0141133] (molecular function) References: PMID:24739148 Sources: RHEA:42652 Note: This activity is present in eukaryotes and is part of the biosynthetic pathway of diphthamide. Note that this is different from the archaeal enzyme, diphthine synthase activity ; GO:0004164 (EC:2.1.1.98), which performs only 3 methylations, producing diphthine. Definition: Catalysis of the reaction: 2-[(3S)-amino-3-carboxypropyl]-L-histidyl-[translation elongation factor 2] + 4 S-adenosyl-L-methionine = diphthine methyl ester-[translation elongation factor 2] + 3 H+ + 4 S-adenosyl-L-homocysteine. Relationships: is a type of protein methyltransferase activity [GO:0008276]; is a type of S-adenosylmethionine-dependent methyltransferase activity [GO:0008757]